amino-acid betaine catabolic process [GO:0006579] (biological process) Definition: The chemical reactions and pathways resulting in the breakdown of any betaine, the N-trimethyl derivative of an amino acid. Subtypes: GO:0019504, glycine betaine catabolic process [GO:0031457], carnitine catabolic process [GO:0042413], ergothioneine catabolic process [GO:0052700] Sources: GOC:mah, ISBN:0198506732 Relationships: is a type of amino-acid betaine metabolic process [GO:0006577]; is a type of modified amino acid catabolic process [GO:0042219] Also known as: betaine breakdown, betaine catabolic process, betaine catabolism, betaine degradation